{
  "gene_name": "N-alpha-acetyltransferase 10",
  "gene": "UniProtKB:P41227",
  "gene_symbol": "NAA10",
  "term_label": "Unknown biological process",
  "term_id": "UNKNOWN:0002"
}